{
  "gene_symbol": "ZNF700",
  "term_label": "DNA-binding transcription factor activity, RNA polymerase II-specific",
  "term_id": "GO:0000981",
  "gene_name": "Zinc finger protein 700",
  "gene": "UniProtKB:Q9H0M5"
}